{
  "term_label": "Unknown molecular function",
  "gene_symbol": "GOLGA8S",
  "gene": "UniProtKB:H3BPF8",
  "term_id": "UNKNOWN:0001",
  "gene_name": "Golgin subfamily A member 8S"
}